deoxyribodipyrimidine endonucleosidase activity [GO:0033959] (molecular function) Also known as: endonuclease V activity, PD-DNA glycosylase activity, T4-induced UV endonuclease activity, deoxy-D-ribocyclobutadipyrimidine polynucleotidodeoxyribohydrolase activity, deoxyribonucleate pyrimidine dimer glycosidase activity, pyrimidine dimer DNA glycosylase activity, pyrimidine dimer DNA-glycosylase activity Definition: Catalysis of the cleavage of the N-glycosidic bond between the 5'-pyrimidine residue in cyclobutadipyrimidine (in DNA) and the corresponding deoxy-D-ribose residue. Relationships: is a type of hydrolase activity, hydrolyzing N-glycosyl compounds [GO:0016799]; is a type of catalytic activity, acting on DNA [GO:0140097] Sources: EC:3.2.2.17